{
  "gene_symbol": "AGBL2",
  "term_id": "GO:0004181",
  "gene_name": "Cytosolic carboxypeptidase 2",
  "gene": "UniProtKB:Q5U5Z8",
  "term_label": "metallocarboxypeptidase activity"
}